{
  "term_label": "D-mannose binding",
  "gene_symbol": "ASGR1",
  "gene": "UniProtKB:P07306",
  "gene_name": "Asialoglycoprotein receptor 1",
  "term_id": "GO:0005537"
}